{
  "term_id": "UNKNOWN:0001",
  "gene": "UniProtKB:O97980",
  "gene_symbol": "HMHB1",
  "gene_name": "Minor histocompatibility protein HB-1",
  "term_label": "Unknown molecular function"
}